{
  "term_id": "UNKNOWN:0003",
  "gene_name": "S phase cyclin A-associated protein in the endoplasmic reticulum",
  "gene": "UniProtKB:Q9BY12",
  "gene_symbol": "SCAPER",
  "term_label": "Unknown cellular component"
}